{
  "term_id": "UNKNOWN:0003",
  "term_label": "Unknown cellular component",
  "gene_symbol": "CLEC19A",
  "gene_name": "C-type lectin domain family 19 member A",
  "gene": "UniProtKB:Q6UXS0"
}